{
  "term_label": "inositol trisphosphate phosphatase activity",
  "term_id": "GO:0046030",
  "gene_symbol": "INPP5K",
  "gene_name": "Inositol polyphosphate 5-phosphatase K",
  "gene": "UniProtKB:Q9BT40"
}